{
  "gene_name": "HHIP-like protein 2",
  "term_label": "Unknown biological process",
  "gene_symbol": "HHIPL2",
  "gene": "UniProtKB:Q6UWX4",
  "term_id": "UNKNOWN:0002"
}